RNA modification [GO:0009451] (biological process) Definition: The covalent alteration of one or more nucleotides within an RNA molecule to produce an RNA molecule with a sequence that differs from that coded genetically. Sources: GOC:go_curators, ISBN:1555811337 Note: The term 'RNA editing' (GO:0016547) was merged into 'RNA modification' (GO:0009451) on the basis of statements in the preface of Modification and Editing of RNA (ISBN:1555811337) that there is no clear distinction between modification and editing. Also known as: RNA editing Relationships: is a type of RNA metabolic process [GO:0016070]; is a type of macromolecule modification [GO:0043412] Subtypes: rRNA modification [GO:0000154], RNA methylation [GO:0001510], pseudouridine synthesis [GO:0001522], tRNA modification [GO:0006400], GO:0016553, GO:0016556, GO:0035513, snRNA modification [GO:0040031], RNA nucleotide insertion [GO:0070705], RNA nucleotide deletion [GO:0070706], GO:1900864, chloroplast RNA modification [GO:1900865], RNA acetylation [GO:1990884]